endoplasmic reticulum unfolded protein response [GO:0030968] (biological process) Note: Note that this term should not be confused with 'response to unfolded protein ; GO:0006986', which refers to any response to the presence of unfolded proteins anywhere in the cell or in multicellular organism. Subtypes: GO:0036498, PERK-mediated unfolded protein response [GO:0036499], GO:0036500 Definition: The series of molecular signals generated as a consequence of the presence of unfolded proteins in the endoplasmic reticulum (ER) or other ER-related stress; results in changes in the regulation of transcription and translation. Relationships: is a type of response to endoplasmic reticulum stress [GO:0034976]; is a type of intracellular signal transduction [GO:0035556]; is part of GO:0034620 References: PMID:12042763 Sources: GOC:mah Regulation: regulated by regulation of endoplasmic reticulum unfolded protein response [GO:1900101]; negatively regulated by negative regulation of endoplasmic reticulum unfolded protein response [GO:1900102]; RO_0002213 by GO:1900103 Also known as: ER unfolded protein response, erUPR, SREBP-mediated signalling pathway